{
  "gene": "UniProtKB:Q9UNE2",
  "gene_name": "Rab effector Noc2",
  "gene_symbol": "RPH3AL",
  "term_label": "synapse",
  "term_id": "GO:0045202"
}